macrophage chemotaxis [GO:0048246] (biological process) Definition: The movement of a macrophage in response to an external stimulus. Sources: GOC:jid Regulation: regulated by GO:0010758; positively regulated by positive regulation of macrophage chemotaxis [GO:0010759]; negatively regulated by negative regulation of macrophage chemotaxis [GO:0010760] Relationships: is a type of GO:0030595; is a type of macrophage migration [GO:1905517]